positive regulation of translational frameshifting [GO:2001126] (biological process) Relationships: is a type of positive regulation of translational elongation [GO:0045901]; is a type of regulation of translational frameshifting [GO:2001124]; positively regulates translational frameshifting [GO:0006452] Definition: Any process that activates or increases the frequency, rate or extent of translational frameshifting. Sources: GOC:obol